{
  "term_id": "GO:0005516",
  "gene_name": "Protein phosphatase 3 catalytic subunit alpha",
  "gene": "UniProtKB:Q08209",
  "gene_symbol": "PPP3CA",
  "term_label": "calmodulin binding"
}